{
  "term_id": "GO:0005829",
  "gene_name": "Rho GTPase-activating protein 17",
  "gene_symbol": "ARHGAP17",
  "term_label": "cytosol",
  "gene": "UniProtKB:Q68EM7"
}